{
  "term_label": "negative regulation of DNA recombination",
  "gene_name": "Histone H1.4",
  "term_id": "GO:0045910",
  "gene_symbol": "H1-4",
  "gene": "UniProtKB:P10412"
}